rubredoxin-NADP+ reductase activity [GO:0015046] (molecular function) Sources: RHEA:13949 Definition: Catalysis of the reaction: 2 reduced [rubredoxin] + NADP+ + H+ = 2 oxidized [rubredoxin] + NADPH. Relationships: is a type of rubredoxin-NAD(P)H reductase activity [GO:0015045]